{
  "gene_name": "Endoplasmin",
  "gene_symbol": "HSP90B1",
  "gene": "UniProtKB:P14625",
  "term_label": "ATP binding",
  "term_id": "GO:0005524"
}